negative regulation of mitochondrial fusion [GO:0010637] (BP) Definition: Any process that decreases the frequency, rate or extent of merging of two or more mitochondria within a cell to form a single compartment. Sources: GOC:dph, GOC:tb Relationships: is a type of regulation of mitochondrial fusion [GO:0010635]; is a type of negative regulation of organelle organization [GO:0010639]; is a type of GO:0051093; RO_0002212 GO:0008053